{
  "term_id": "GO:0003341",
  "gene": "UniProtKB:Q8NA47",
  "gene_symbol": "CCDC63",
  "term_label": "cilium movement",
  "gene_name": "Coiled-coil domain-containing protein 63"
}